{
  "term_label": "regulation of transcription by RNA polymerase II",
  "term_id": "GO:0006357",
  "gene": "UniProtKB:O60393",
  "gene_symbol": "NOBOX",
  "gene_name": "Homeobox protein NOBOX"
}